{
  "gene": "UniProtKB:Q9Y5T5",
  "term_label": "Unknown cellular component",
  "gene_name": "Ubiquitin carboxyl-terminal hydrolase 16",
  "term_id": "UNKNOWN:0003",
  "gene_symbol": "USP16"
}